{
  "term_id": "GO:1901096",
  "term_label": "regulation of autophagosome maturation",
  "gene_symbol": "CLEC16A",
  "gene_name": "Protein CLEC16A",
  "gene": "UniProtKB:Q2KHT3"
}